{
  "term_label": "gap junction channel activity",
  "gene": "UniProtKB:Q8NFK1",
  "term_id": "GO:0005243",
  "gene_name": "Gap junction gamma-3 protein",
  "gene_symbol": "GJC3"
}